{
  "gene": "UniProtKB:Q96JP5",
  "term_id": "GO:0006357",
  "gene_name": "E3 ubiquitin-protein ligase ZFP91",
  "gene_symbol": "ZFP91",
  "term_label": "regulation of transcription by RNA polymerase II"
}